{
  "gene_symbol": "SLC2A9",
  "gene_name": "Solute carrier family 2, facilitated glucose transporter member 9",
  "term_label": "D-glucose transmembrane transporter activity",
  "term_id": "GO:0055056",
  "gene": "UniProtKB:Q9NRM0"
}